{
  "term_label": "proteasome regulatory particle, base subcomplex",
  "term_id": "GO:0008540",
  "gene_name": "26S proteasome regulatory subunit 10B",
  "gene_symbol": "PSMC6",
  "gene": "UniProtKB:P62333"
}